{
  "term_id": "GO:0019911",
  "gene_name": "Noncompact myelin-associated protein",
  "term_label": "structural constituent of myelin sheath",
  "gene_symbol": "NCMAP",
  "gene": "UniProtKB:Q5T1S8"
}